{
  "term_label": "cytoplasm",
  "gene": "UniProtKB:Q16527",
  "gene_name": "Cysteine and glycine-rich protein 2",
  "gene_symbol": "CSRP2",
  "term_id": "GO:0005737"
}